{
  "gene_name": "Importin subunit alpha-1",
  "term_label": "nuclear import signal receptor activity",
  "gene": "UniProtKB:P52292",
  "term_id": "GO:0061608",
  "gene_symbol": "KPNA2"
}